{
  "gene": "UniProtKB:O15243",
  "gene_name": "Leptin receptor gene-related protein",
  "term_label": "late endosome to vacuole transport via multivesicular body sorting pathway",
  "gene_symbol": "LEPROT",
  "term_id": "GO:0032511"
}